{
  "gene_name": "Zinc transporter ZIP5",
  "term_label": "monoatomic cation:bicarbonate symporter activity",
  "gene": "UniProtKB:Q6ZMH5",
  "term_id": "GO:0140410",
  "gene_symbol": "SLC39A5"
}